CD40 receptor complex [GO:0035631] (cellular component) Relationships: is a type of plasma membrane signaling receptor complex [GO:0098802] Definition: A protein complex that contains at least CD40 (a cell surface receptor of the tumour necrosis factor receptor (TNFR) superfamily), and other signaling molecules. References: PMID:20614026, PMID:9221764 Sources: GOC:BHF